{
  "gene_name": "Novel acetylcholine receptor chaperone",
  "term_label": "acetylcholine receptor regulator activity",
  "gene_symbol": "TMEM35A",
  "term_id": "GO:0030548",
  "gene": "UniProtKB:Q53FP2"
}